metanephric pyramids development [GO:0072211] (biological process) Definition: The process whose specific outcome is the progression of the metanephric pyramids over time, from their formation to the mature structures. Metanephric pyramids are the conical masses that constitute the renal medulla in a metanephros; they contain the loops of Henle and the medullary collecting ducts. Sources: GOC:mtg_kidney_jan10 Also known as: metanephric kidney pyramid development, metanephric pyramid development, metanephric renal medulla development, metanephric renal pyramid development Relationships: is_a pyramid development [GO:0072056]; BFO_0000050 metanephros development [GO:0001656]